phytoene catabolic process [GO:1901173] (biological process) Also known as: phytoene breakdown, phytoene catabolism, phytoene degradation Sources: GOC:TermGenie, GOC:yaf, UniPathway:UPA00799 Relationships: is a type of carotene catabolic process [GO:0016121] Definition: The chemical reactions and pathways resulting in the breakdown of phytoene.